erythrocyte maturation [GO:0043249] (BP) Also known as: RBC maturation, red blood cell maturation Sources: GOC:devbiol, GOC:jl Relationships: is a type of GO:0048469; is part of erythrocyte development [GO:0048821] Subtypes: GO:0043354, GO:0043362 Definition: A developmental process, independent of morphogenetic (shape) change, that is required for an erythrocyte to attain its fully functional state.